receptor guanylyl cyclase signaling pathway [GO:0007168] (biological process) Relationships: is a type of GO:0007167 Definition: The series of molecular signals initiated by an extracellular ligand binding to a receptor on the surface of the target cell where the receptor possesses guanylyl cyclase activity, and converts GTP to cGMP upon activation, and ending with the regulation of a downstream cellular process, e.g. transcription. Also known as: cGMP signaling pathway, receptor guanylate cyclase signaling pathway, receptor guanylyl cyclase signalling pathway Regulation: negatively regulated by negative regulation of receptor guanylyl cyclase signaling pathway [GO:0010754] References: PMID:16815030 Sources: GOC:mah, GOC:signaling